I-SMAD binding [GO:0070411] (molecular function) Relationships: is a type of GO:0046332 Definition: Binding to an inhibitory SMAD signaling protein. References: PMID:19114992 Sources: GOC:BHF, GOC:vk